{
  "gene_name": "RNA-binding protein Musashi homolog 2",
  "term_id": "GO:0007417",
  "gene_symbol": "MSI2",
  "term_label": "central nervous system development",
  "gene": "UniProtKB:Q96DH6"
}